{
  "gene": "UniProtKB:Q6P1K1",
  "term_id": "GO:0005765",
  "term_label": "lysosomal membrane",
  "gene_symbol": "SLC48A1",
  "gene_name": "Heme transporter HRG1"
}